regulation of systemic arterial blood pressure mediated by a chemical signal [GO:0003044] (biological process) Definition: The regulation of blood pressure mediated by biochemical signaling: hormonal, autocrine or paracrine. Sources: GOC:mtg_cardio Also known as: blood pressure regulation mediated by a chemical signal Relationships: is a type of regulation of systemic arterial blood pressure [GO:0003073] Subtypes: regulation of systemic arterial blood pressure by hormone [GO:0001990], regulation of systemic arterial blood pressure by norepinephrine-epinephrine [GO:0001993], GO:0003047, GO:0003048, regulation of systemic arterial blood pressure by neurotransmitter [GO:0003070]